{
  "gene_name": "Olfactory receptor 5K2",
  "gene_symbol": "OR5K2",
  "term_label": "olfactory receptor activity",
  "term_id": "GO:0004984",
  "gene": "UniProtKB:Q8NHB8"
}